{
  "gene": "UniProtKB:O75473",
  "gene_symbol": "LGR5",
  "term_label": "Unknown molecular function",
  "term_id": "UNKNOWN:0001",
  "gene_name": "Leucine-rich repeat-containing G-protein coupled receptor 5"
}